{
  "gene_symbol": "VTI1A",
  "gene_name": "Vesicle transport through interaction with t-SNAREs homolog 1A",
  "gene": "UniProtKB:Q96AJ9",
  "term_label": "ER to Golgi transport vesicle membrane",
  "term_id": "GO:0012507"
}